{
  "term_label": "Unknown biological process",
  "term_id": "UNKNOWN:0002",
  "gene_name": "Endonuclease domain-containing 1 protein",
  "gene_symbol": "ENDOD1",
  "gene": "UniProtKB:O94919"
}